glyceraldehyde 3-phosphate:phosphate antiporter activity [GO:0051408] (molecular function) Definition: Enables the transfer of a solute or solutes from one side of a membrane to the other according to the reaction: glyceraldehyde 3-phosphate(out) + phosphate(in) = glyceraldehyde 3-phosphate(in) + phosphate(out). Also known as: glyceraldehyde 3-phosphate:inorganic phosphate antiporter activity Relationships: is a type of triose-phosphate:phosphate antiporter activity [GO:0009670] Sources: GOC:ai